{
  "term_id": "GO:0005085",
  "gene_symbol": "SBF1",
  "term_label": "guanyl-nucleotide exchange factor activity",
  "gene_name": "Myotubularin-related protein 5",
  "gene": "UniProtKB:O95248"
}